{
  "gene_symbol": "PTOV1",
  "gene": "UniProtKB:Q86YD1",
  "term_label": "positive regulation of transcription by RNA polymerase II",
  "gene_name": "Prostate tumor-overexpressed gene 1 protein",
  "term_id": "GO:0045944"
}